positive regulation of seed dormancy process [GO:1902040] (BP) References: PMID:23378449 Sources: GOC:TermGenie Also known as: up regulation of seed dormancy process, up-regulation of seed dormancy process, upregulation of seed dormancy process, activation of seed dormancy process, activation of seed dormancy, positive regulation of seed dormancy, up regulation of seed dormancy, up-regulation of seed dormancy, upregulation of seed dormancy Relationships: is a type of positive regulation of developmental process [GO:0051094]; is a type of positive regulation of multicellular organismal process [GO:0051240]; is a type of GO:2000033; is a type of positive regulation of reproductive process [GO:2000243]; positively regulates seed dormancy process [GO:0010162] Definition: Any process that activates or increases the frequency, rate or extent of seed dormancy process.